diaminobutyrate decarboxylase activity [GO:0033983] (molecular function) Definition: Catalysis of the reaction: L-2,4-diaminobutyrate + H+ = 1,3-diaminopropane + CO2. Sources: EC:4.1.1.86, RHEA:15689 Relationships: is a type of GO:0016831 Also known as: DABA DC, L-2,4-diaminobutanoate carboxy-lyase (propane-1,3-diamine-forming) activity, L-2,4-diaminobutanoate carboxy-lyase activity, L-2,4-diaminobutyrate decarboxylase activity